respiratory electron transport chain [GO:0022904] (biological process) Also known as: electron transfer, 6-phosphofructokinase reduction, dihydrobiopterin reduction, dihydrolipoamide reduction, dihydrolipoylprotein reduction, dihydropteridine reduction, other pathways of electron transport, oxidized glutathione reduction, protein-disulfide reduction Definition: A process in which a series of electron carriers operate together to transfer electrons from donors such as NADH and FADH2 to any of several different terminal electron acceptors to generate a transmembrane electrochemical gradient. Relationships: is a type of electron transport chain [GO:0022900]; is part of cellular respiration [GO:0045333] Sources: GOC:mtg_electron_transport, ISBN:0716720094 Subtypes: chlororespiration [GO:0010478], anaerobic electron transport chain [GO:0019645], aerobic electron transport chain [GO:0019646], plasma membrane electron transport, NADH to quinone [GO:0030965], ATP synthesis coupled electron transport [GO:0042773]